{
  "gene_name": "CCN family member 1",
  "term_id": "GO:0007165",
  "term_label": "signal transduction",
  "gene": "UniProtKB:O00622",
  "gene_symbol": "CCN1"
}